{
  "term_id": "GO:0007608",
  "term_label": "sensory perception of smell",
  "gene_symbol": "OR5I1",
  "gene": "UniProtKB:Q13606",
  "gene_name": "Olfactory receptor 5I1"
}